{
  "gene_symbol": "PPP1R11",
  "term_id": "GO:0008157",
  "gene": "UniProtKB:O60927",
  "gene_name": "E3 ubiquitin-protein ligase PPP1R11",
  "term_label": "protein phosphatase 1 binding"
}